{
  "term_id": "GO:0040011",
  "gene_symbol": "WDR1",
  "term_label": "locomotion",
  "gene": "UniProtKB:O75083",
  "gene_name": "WD repeat-containing protein 1"
}